{
  "term_label": "anaphase-promoting complex",
  "gene": "UniProtKB:Q9UM13",
  "gene_symbol": "ANAPC10",
  "gene_name": "Anaphase-promoting complex subunit 10",
  "term_id": "GO:0005680"
}